{
  "term_label": "pattern recognition receptor activity",
  "gene": "UniProtKB:Q9BXN2",
  "term_id": "GO:0038187",
  "gene_name": "C-type lectin domain family 7 member A",
  "gene_symbol": "CLEC7A"
}